{
  "term_id": "GO:0000175",
  "term_label": "3'-5'-RNA exonuclease activity",
  "gene_name": "DIS3-like exonuclease 1",
  "gene": "UniProtKB:Q8TF46",
  "gene_symbol": "DIS3L"
}